agglutination involved in conjugation with mutual genetic exchange [GO:0000758] (biological process) Also known as: agglutination involved in conjugation without cellular fusion, sexual flocculation Definition: The aggregation or adhesion of compatible mating types via complementary cell-cell interactions during conjugation without cellular fusion of a unicellular organism. Sources: GOC:elh Relationships: is a type of biological process involved in intraspecies interaction between organisms [GO:0051703]; is a type of GO:0140039; is part of response to pheromone regulating conjugation with mutual genetic exchange [GO:0000756]